{
  "term_id": "GO:0005938",
  "gene_name": "CAP-Gly domain-containing linker protein 4",
  "gene": "UniProtKB:Q8N3C7",
  "gene_symbol": "CLIP4",
  "term_label": "cell cortex"
}